{
  "term_id": "UNKNOWN:0003",
  "gene_symbol": "DNAJC4",
  "gene_name": "DnaJ homolog subfamily C member 4",
  "gene": "UniProtKB:Q9NNZ3",
  "term_label": "Unknown cellular component"
}